{
  "term_label": "apical plasma membrane",
  "term_id": "GO:0016324",
  "gene_name": "Sodium-dependent phosphate transport protein 2A",
  "gene": "UniProtKB:Q06495",
  "gene_symbol": "SLC34A1"
}